{
  "gene_symbol": "DNMBP",
  "gene": "UniProtKB:Q6XZF7",
  "term_label": "guanyl-nucleotide exchange factor activity",
  "gene_name": "Dynamin-binding protein",
  "term_id": "GO:0005085"
}